{
  "term_label": "DNA-binding transcription factor activity",
  "term_id": "GO:0003700",
  "gene": "UniProtKB:Q9NVV9",
  "gene_symbol": "THAP1",
  "gene_name": "THAP domain-containing protein 1"
}